{
  "term_label": "nucleus",
  "gene": "UniProtKB:P41161",
  "gene_name": "ETS translocation variant 5",
  "term_id": "GO:0005634",
  "gene_symbol": "ETV5"
}